{
  "gene_symbol": "GON4L",
  "term_label": "transcription coregulator activity",
  "gene_name": "GON-4-like protein",
  "term_id": "GO:0003712",
  "gene": "UniProtKB:Q3T8J9"
}